cloaca development [GO:0035844] (biological process) Sources: GOC:dgh, ISBN:0582227089 Relationships: is a type of anatomical structure development [GO:0048856]; is part of urogenital system development [GO:0001655]; is part of digestive tract morphogenesis [GO:0048546] Definition: The process whose specific outcome is the progression of the cloaca over time, from it's formation to the mature structure. The cloaca is the common chamber into which intestinal, genital and urinary canals open in vertebrates. Also known as: cloacal development